{
  "term_label": "RNA nuclease activity",
  "gene_name": "Ribonuclease 4",
  "term_id": "GO:0004540",
  "gene": "UniProtKB:P34096",
  "gene_symbol": "RNASE4"
}